iron coordination entity transport [GO:1901678] (BP) Sources: GOC:TermGenie, GOC:pr Definition: The directed movement of an iron coordination entity into, out of or within a cell, or between cells, by means of some agent such as a transporter or pore. Subtypes: heme transport [GO:0015886], siderophore transport [GO:0015891], siderophore-iron import into cell [GO:0033214], iron-sulfur cluster transmembrane transport [GO:1902497] Relationships: is a type of iron ion transport [GO:0006826]